{
  "gene": "UniProtKB:Q9H489",
  "term_id": "GO:0003682",
  "term_label": "chromatin binding",
  "gene_symbol": "TSPY26P",
  "gene_name": "Putative testis-specific Y-encoded-like protein 3"
}